{
  "gene_name": "Disintegrin and metalloproteinase domain-containing protein 30",
  "gene_symbol": "ADAM30",
  "term_label": "external side of plasma membrane",
  "term_id": "GO:0009897",
  "gene": "UniProtKB:Q9UKF2"
}